{
  "term_label": "ubiquitin-dependent protein catabolic process",
  "gene": "UniProtKB:Q00987",
  "gene_symbol": "MDM2",
  "term_id": "GO:0006511",
  "gene_name": "E3 ubiquitin-protein ligase Mdm2"
}